{
  "gene_symbol": "COBL",
  "term_label": "ruffle",
  "term_id": "GO:0001726",
  "gene_name": "Protein cordon-bleu",
  "gene": "UniProtKB:O75128"
}